{
  "gene": "UniProtKB:P07947",
  "gene_symbol": "YES1",
  "gene_name": "Tyrosine-protein kinase Yes",
  "term_id": "GO:0005102",
  "term_label": "signaling receptor binding"
}